negative regulation of adaptive immune response [GO:0002820] (biological process) Subtypes: negative regulation of adaptive immune response based on somatic recombination of immune receptors built from immunoglobulin superfamily domains [GO:0002823], negative regulation of adaptive immune memory response [GO:1905675], negative regulation of adaptive immune effector response [GO:1905678] Sources: GOC:add Relationships: is a type of regulation of adaptive immune response [GO:0002819]; is_a GO:0050777; negatively regulates GO:0002250 Also known as: down regulation of adaptive immune response, down-regulation of adaptive immune response, downregulation of adaptive immune response, inhibition of adaptive immune response Definition: Any process that stops, prevents, or reduces the frequency, rate, or extent of an adaptive immune response.